{
  "term_id": "UNKNOWN:0002",
  "gene": "UniProtKB:Q9GZU0",
  "term_label": "Unknown biological process",
  "gene_name": "Uncharacterized protein C6orf62",
  "gene_symbol": "C6orf62"
}